phloroisovalerophenone synthase activity [GO:0050634] (MF) Definition: Catalysis of the reaction: isovaleryl-CoA + 3 malonyl-CoA = 4 CoASH + 3 CO2 + 3-methyl-1-(2,4,6-trihydroxyphenyl)butan-1-one. Relationships: is a type of acyltransferase activity, transferring groups other than amino-acyl groups [GO:0016747] Sources: EC:2.3.1.156, MetaCyc:2.3.1.156-RXN Also known as: 3-methyl-1-(trihydroxyphenyl)butan-1-one synthase activity, isovaleryl-CoA:malonyl-CoA acyltransferase activity, valerophenone synthase activity